{
  "gene_symbol": "CDH5",
  "term_label": "beta-catenin binding",
  "gene": "UniProtKB:P33151",
  "term_id": "GO:0008013",
  "gene_name": "Cadherin-5"
}